negative regulation of long-chain fatty acid import across plasma membrane [GO:0010748] (biological process) Definition: Any process that decreases the rate, frequency or extent of plasma membrane long-chain fatty acid transport. Plasma membrane long-chain fatty acid transport is the directed movement of long-chain fatty acids across the plasma membrane. Also known as: negative regulation of plasma membrane long-chain fatty acid transport Relationships: is a type of regulation of long-chain fatty acid import across plasma membrane [GO:0010746]; is a type of GO:0034763; is a type of negative regulation of long-chain fatty acid import into cell [GO:0140213]; negatively regulates GO:0015911 Sources: GOC:BHF, GOC:dph, GOC:tb